{
  "term_id": "GO:0016477",
  "gene_name": "Cadherin-9",
  "gene_symbol": "CDH9",
  "term_label": "cell migration",
  "gene": "UniProtKB:Q9ULB4"
}